{
  "gene": "UniProtKB:Q9Y261",
  "gene_name": "Hepatocyte nuclear factor 3-beta",
  "gene_symbol": "FOXA2",
  "term_id": "GO:0000978",
  "term_label": "RNA polymerase II cis-regulatory region sequence-specific DNA binding"
}